{
  "gene_name": "CDK5 and ABL1 enzyme substrate 2",
  "gene": "UniProtKB:Q9BTV7",
  "term_id": "UNKNOWN:0002",
  "term_label": "Unknown biological process",
  "gene_symbol": "CABLES2"
}